{
  "gene_name": "Golgin subfamily A member 8C",
  "gene": "UniProtKB:A6NN73",
  "term_id": "GO:0005801",
  "gene_symbol": "GOLGA8CP",
  "term_label": "cis-Golgi network"
}